{
  "gene_symbol": "RPP14",
  "gene_name": "Ribonuclease P protein subunit p14",
  "gene": "UniProtKB:O95059",
  "term_id": "GO:0005730",
  "term_label": "nucleolus"
}